{
  "gene_symbol": "CFAP90",
  "gene_name": "Cilia- and flagella-associated protein 90",
  "term_label": "Unknown cellular component",
  "term_id": "UNKNOWN:0003",
  "gene": "UniProtKB:A4QMS7"
}